mitochondrial prohibitin complex [GO:0035632] (cellular component) References: PMID:12237468, PMID:21164222 Sources: GOC:kmv Definition: A complex composed of two proteins, prohibitin 1 and prohibitin 2 (PHB1/PHB-1 and PHB2/PHB-2) that is highly conserved amongst eukaryotes and associated with the inner mitochondrial membrane. The mitochondrial prohibitin complex is a macromolecular supercomplex composed of repeating heterodimeric subunits of PHB1 and PHB2. The mitochondrial prohibitin complex plays a role in a number of biological processes, including mitochondrial biogenesis and function, development, replicative senescence, and cell death. Also known as: mitochondrial inner membrane prohibitin complex Relationships: is a type of inner mitochondrial membrane protein complex [GO:0098800]